{
  "term_label": "regulation of transcription by RNA polymerase II",
  "gene_symbol": "ZGLP1",
  "gene": "UniProtKB:P0C6A0",
  "gene_name": "GATA-type zinc finger protein 1",
  "term_id": "GO:0006357"
}